{
  "term_id": "UNKNOWN:0002",
  "term_label": "Unknown biological process",
  "gene_name": "Uncharacterized protein C1orf167",
  "gene_symbol": "C1orf167",
  "gene": "UniProtKB:Q5SNV9"
}